{
  "gene_symbol": "DDX56",
  "gene_name": "Probable ATP-dependent RNA helicase DDX56",
  "term_label": "Unknown biological process",
  "gene": "UniProtKB:Q9NY93",
  "term_id": "UNKNOWN:0002"
}